plastid thylakoid membrane [GO:0055035] (cellular component) Relationships: is a type of GO:0042170; is a type of thylakoid membrane [GO:0042651]; is part of plastid thylakoid [GO:0031976] Subtypes: GO:0009535, cyanelle thylakoid membrane [GO:0033115], prothylakoid membrane [GO:0042650] Definition: The lipid bilayer membrane of any thylakoid within a plastid. Sources: GOC:jid, GOC:rph